{
  "gene_name": "F-box only protein 17",
  "term_id": "GO:0031146",
  "gene_symbol": "FBXO17",
  "term_label": "SCF-dependent proteasomal ubiquitin-dependent protein catabolic process",
  "gene": "UniProtKB:Q96EF6"
}